{
  "term_label": "RNA polymerase II cis-regulatory region sequence-specific DNA binding",
  "gene_name": "POU domain, class 5, transcription factor 2",
  "gene_symbol": "POU5F2",
  "term_id": "GO:0000978",
  "gene": "UniProtKB:Q8N7G0"
}